{
  "gene_symbol": "SMIM28",
  "term_id": "UNKNOWN:0002",
  "gene": "UniProtKB:A0A1B0GU29",
  "term_label": "Unknown biological process",
  "gene_name": "Small integral membrane protein 28"
}